{
  "term_id": "GO:0022848",
  "gene_symbol": "CHRNB1",
  "gene_name": "Acetylcholine receptor subunit beta",
  "term_label": "acetylcholine-gated monoatomic cation-selective channel activity",
  "gene": "UniProtKB:P11230"
}